{
  "gene": "UniProtKB:Q9NWV4",
  "gene_symbol": "CZIB",
  "term_id": "UNKNOWN:0003",
  "gene_name": "CXXC motif containing zinc binding protein",
  "term_label": "Unknown cellular component"
}